{
  "term_id": "GO:0030336",
  "gene_symbol": "RAP2B",
  "gene_name": "Ras-related protein Rap-2b",
  "gene": "UniProtKB:P61225",
  "term_label": "negative regulation of cell migration"
}